plasmodesmata-mediated intercellular transport [GO:0010497] (biological process) Relationships: is a type of intercellular transport [GO:0010496] Definition: The movement of substances between cells via plasmodesmata. Plasmodesmata is a fine cytoplasmic channel, found in all higher plants, that connects the cytoplasm of one cell to that of an adjacent cell. Also known as: plasmodesma-mediated cell-to-cell transport, plasmodesma-mediated intercellular transport, plasmodesmata-mediated cell-to-cell transport, single organism plasmodesmata-mediated intercellular transport, single-organism plasmodesmata-mediated intercellular transport References: PMID:17601829